muscle organ morphogenesis [GO:0048644] (biological process) Definition: The process in which the anatomical structures of muscle are generated and organized. Subtypes: diaphragm morphogenesis [GO:0060540] Sources: GOC:jid Relationships: is a type of animal organ morphogenesis [GO:0009887]; is part of muscle organ development [GO:0007517]